{
  "gene_symbol": "TNS4",
  "term_label": "Unknown biological process",
  "gene": "UniProtKB:Q8IZW8",
  "term_id": "UNKNOWN:0002",
  "gene_name": "Tensin-4"
}